GTPase binding [GO:0051020] (molecular function) Sources: GOC:ai Subtypes: GO:0031267 Definition: Binding to a GTPase, any enzyme that catalyzes the hydrolysis of GTP. Relationships: is a type of enzyme binding [GO:0019899]